single-strand break-containing DNA binding [GO:1990165] (molecular function) Also known as: SSB-containing DNA binding, single-strand break-containing damaged DNA binding References: PMID:21984210 Sources: GOC:al Definition: Binding to damaged DNA containing single-strand breaks (SSBs). Relationships: is a type of damaged DNA binding [GO:0003684]